{
  "term_id": "GO:0000978",
  "gene_name": "Homeobox protein Nkx-2.5",
  "gene_symbol": "NKX2-5",
  "term_label": "RNA polymerase II cis-regulatory region sequence-specific DNA binding",
  "gene": "UniProtKB:P52952"
}